{
  "term_label": "chromatin binding",
  "term_id": "GO:0003682",
  "gene_symbol": "ENY2",
  "gene_name": "Transcription and mRNA export factor ENY2",
  "gene": "UniProtKB:Q9NPA8"
}